{
  "gene_name": "L-dopachrome tautomerase",
  "gene": "UniProtKB:P40126",
  "term_id": "GO:0002052",
  "gene_symbol": "DCT",
  "term_label": "positive regulation of neuroblast proliferation"
}